{
  "gene_name": "Nuclear RNA export factor 5",
  "term_label": "RNA binding",
  "term_id": "GO:0003723",
  "gene": "UniProtKB:Q9H1B4",
  "gene_symbol": "NXF5"
}